{
  "gene": "UniProtKB:Q96RY5",
  "gene_name": "Protein cramped-like",
  "term_id": "GO:0007389",
  "gene_symbol": "CRAMP1",
  "term_label": "pattern specification process"
}